{
  "gene": "UniProtKB:O75439",
  "gene_name": "Mitochondrial-processing peptidase subunit beta",
  "term_label": "mitochondrial processing peptidase complex",
  "term_id": "GO:0017087",
  "gene_symbol": "PMPCB"
}